{
  "gene_symbol": "CDC42BPG",
  "gene_name": "Serine_threonine-protein kinase MRCK gamma",
  "term_id": "GO:0031032",
  "gene": "UniProtKB:Q6DT37",
  "term_label": "actomyosin structure organization"
}